{
  "term_id": "GO:0030170",
  "gene_name": "Serine racemase",
  "gene_symbol": "SRR",
  "term_label": "pyridoxal phosphate binding",
  "gene": "UniProtKB:Q9GZT4"
}